zymogen granule [GO:0042588] (cellular component) Relationships: is a type of secretory granule [GO:0030141] Sources: GOC:jl, ISBN:0198506732 Definition: A membrane-bounded, cytoplasmic secretory granule found in enzyme-secreting cells and visible by light microscopy. Contain zymogen, an inactive enzyme precursor, often of a digestive enzyme.